{
  "gene": "UniProtKB:Q8IXI2",
  "gene_symbol": "RHOT1",
  "term_id": "GO:0005525",
  "gene_name": "Mitochondrial Rho GTPase 1",
  "term_label": "GTP binding"
}